{
  "term_id": "UNKNOWN:0001",
  "gene_name": "THO complex subunit 3",
  "gene_symbol": "THOC3",
  "term_label": "Unknown molecular function",
  "gene": "UniProtKB:Q96J01"
}